{
  "gene_symbol": "MRTFB",
  "term_id": "GO:0005634",
  "gene_name": "Myocardin-related transcription factor B",
  "term_label": "nucleus",
  "gene": "UniProtKB:Q9ULH7"
}